galactosamine-6-phosphate isomerase activity [GO:0043877] (molecular function) Relationships: is a type of GO:0016861 Also known as: galactosamine-6-phosphate deaminase activity, AgaI References: PMID:10931310 Definition: Catalysis of the reaction: D-galactosamine 6-phosphate + H2O = D-tagatose 6-phosphate + NH3. Note: This function is part of the pathway of N-acetyl-galactosamine and galactosamine utilization.